transcriptional attenuation by ribosome [GO:0031556] (biological process) Also known as: ribosome-mediated transcriptional attenuation Sources: GOC:dh, GOC:mlg, ISBN:0198542682 Definition: A type of transcriptional regulation at the level of early termination. This process can occur only in prokaryotes, where transcription of an operon into messenger RNA and translation of that mRNA into polypeptides occur simultaneously. The general principle is that alternative mRNA secondary structures occur under different physiological conditions such as available amount of a particular amino acid. One set of conditions favors early termination of transcription. In the classic example of the trp biosynthesis operon, translation of the gene for a short, trp-containing polypeptide called the trp operon leader peptide pauses either at a trp codon (if tryptophan is scarce) or the stop codon (if trp is readily available). In the former situation transcription continues, but in the latter a Rho-independent terminator forms and reduces, or attenuates, expression of the tryptophan biosynthesis genes. Although the polypeptides encoded by leader peptide genes appear not to be stable once their translation is complete, it is suggested by recent studies that their nascent polypeptide chains interact specifically with ribosomes, specific uncharged tRNAs, or other cellular components to inhibit release at the stop codon and improve the function of transcriptional attenuation as a regulatory switch. Relationships: is a type of transcriptional attenuation [GO:0031555]